{
  "gene": "UniProtKB:P49407",
  "term_label": "cytosol",
  "gene_name": "Beta-arrestin-1",
  "term_id": "GO:0005829",
  "gene_symbol": "ARRB1"
}